{
  "gene_symbol": "GRIA4",
  "gene_name": "Glutamate receptor 4",
  "term_id": "GO:0050804",
  "term_label": "modulation of chemical synaptic transmission",
  "gene": "UniProtKB:P48058"
}